{
  "gene_symbol": "ATP12A",
  "term_label": "sodium ion export across plasma membrane",
  "gene_name": "Potassium-transporting ATPase alpha chain 2",
  "term_id": "GO:0036376",
  "gene": "UniProtKB:P54707"
}